{
  "term_id": "GO:0071013",
  "gene": "UniProtKB:P62314",
  "gene_symbol": "SNRPD1",
  "gene_name": "Small nuclear ribonucleoprotein Sm D1",
  "term_label": "catalytic step 2 spliceosome"
}